{
  "gene": "UniProtKB:Q8IY92",
  "gene_symbol": "SLX4",
  "term_id": "GO:0033557",
  "gene_name": "Structure-specific endonuclease subunit SLX4",
  "term_label": "Slx1-Slx4 complex"
}